positive regulation of skeletal muscle contraction by regulation of release of sequestered calcium ion [GO:0014810] (biological process) Relationships: is a type of regulation of skeletal muscle contraction by regulation of release of sequestered calcium ion [GO:0014809]; is a type of positive regulation of striated muscle contraction [GO:0045989] Sources: GOC:mtg_muscle Definition: Any process that activates, maintains or increases the frequency, rate or extent of skeletal muscle contraction via the regulation of the release of sequestered calcium ion by sarcoplasmic reticulum into cytosol. The sarcoplasmic reticulum is the endoplasmic reticulum of striated muscle, specialised for the sequestration of calcium ions that are released upon receipt of a signal relayed by the T tubules from the neuromuscular junction.